copper ion transmembrane transporter complex [GO:1903113] (cellular component) Note: An example of this is CusA in E. coli (UniProt symbol P38054) in PMID:23122209 (inferred from direct assay). Definition: A protein complex which is capable of copper ion transmembrane transporter activity. Relationships: is a type of transmembrane transporter complex [GO:1902495] References: PMID:23122209 Sources: GOC:TermGenie, GOC:bhm, GO_REF:0000088 Subtypes: Cus cation efflux complex [GO:1990398]